disruption of plasma membrane integrity in another organism [GO:0051673] (BP) Sources: GOC:ai Relationships: is a type of GO:0140975 Definition: The disruption of the cell membrane of another organism, leading to damage or temporary subversion of the membrane. Also known as: disruption by organism of host cell membrane, disruption of membrane integrity in another organism, membrane disruption in other organism, perturbation of plasma membrane integrity in another organism, cytolysis, by membrane disruption, in other organism, disruption by virus of host cell membrane, membrane disruption in another organism Subtypes: pore formation in membrane of another organism [GO:0035915]